{
  "gene_symbol": "C1GALT1C1L",
  "gene_name": "C1GALT1-specific chaperone 1-like protein",
  "gene": "UniProtKB:P0DN25",
  "term_id": "UNKNOWN:0003",
  "term_label": "Unknown cellular component"
}